{
  "gene_name": "Protein phosphatase 1 regulatory subunit 29",
  "term_label": "plasma membrane",
  "gene": "UniProtKB:Q5R3F8",
  "term_id": "GO:0005886",
  "gene_symbol": "ELFN2"
}